regulation of amacrine cell differentiation [GO:1902869] (biological process) References: PMID:16872597 Sources: GOC:TermGenie, GOC:mr, GO_REF:0000058 Relationships: is a type of GO:0045664; regulates amacrine cell differentiation [GO:0035881] Also known as: regulation of amacrine neuron differentiation Definition: Any process that modulates the frequency, rate or extent of amacrine cell differentiation. Subtypes: negative regulation of amacrine cell differentiation [GO:1902870], positive regulation of amacrine cell differentiation [GO:1902871]